{
  "term_id": "UNKNOWN:0002",
  "term_label": "Unknown biological process",
  "gene": "UniProtKB:Q9BY71",
  "gene_symbol": "LRRC3",
  "gene_name": "Leucine-rich repeat-containing protein 3"
}